{
  "term_label": "cytokine-mediated signaling pathway",
  "gene_symbol": "IRF5",
  "gene": "UniProtKB:Q13568",
  "term_id": "GO:0019221",
  "gene_name": "Interferon regulatory factor 5"
}